{
  "gene_symbol": "ZNF549",
  "gene": "UniProtKB:Q6P9A3",
  "term_id": "GO:0000981",
  "gene_name": "Zinc finger protein 549",
  "term_label": "DNA-binding transcription factor activity, RNA polymerase II-specific"
}